regulation of amyloid-beta clearance [GO:1900221] (biological process) Relationships: is_a GO:0051239; regulates GO:0097242 Also known as: regulation of beta-amyloid clearance Subtypes: negative regulation of amyloid-beta clearance [GO:1900222], positive regulation of amyloid-beta clearance [GO:1900223] Sources: GOC:BHF, GOC:TermGenie Definition: Any process that modulates the frequency, rate or extent of amyloid-beta clearance.